dendrite arborization [GO:0140059] (biological process) Relationships: is a type of dendrite morphogenesis [GO:0048813]; is a type of neuron projection arborization [GO:0140058] Subtypes: basal dendrite arborization [GO:0150020], apical dendrite arborization [GO:0150023] Definition: The process in which the anatomical structures of a dendritic tree are generated and organized into dendritic branches. References: PMID:23270857 Sources: GOC:aruk, GOC:bc